alpha9-beta1 integrin-VEGF-A complex [GO:0071122] (cellular component) Definition: A protein complex that consists of an alpha9-beta1 integrin complex bound to vascular endothelial growth factor A. References: PMID:17363377 Also known as: ITGA9-ITGB1-VEGFA complex Relationships: is a type of GO:0098797